{
  "term_id": "UNKNOWN:0001",
  "gene_symbol": "YIPF2",
  "gene": "UniProtKB:Q9BWQ6",
  "gene_name": "Protein YIPF2",
  "term_label": "Unknown molecular function"
}